detoxification [GO:0098754] (biological process) Sources: GOC:dos Relationships: is a type of biological_process [GO:0008150]; is part of response to toxic substance [GO:0009636] Definition: Any process that reduces or removes the toxicity of a toxic substance. These may include transport of the toxic substance away from sensitive areas and to compartments or complexes whose purpose is sequestration of the toxic substance. Subtypes: toxin catabolic process [GO:0009407], mycothiol-dependent detoxification [GO:0010127], detoxification of nitrogen compound [GO:0051410], detoxification of inorganic compound [GO:0061687], detoxification of arsenic-containing substance [GO:0071722], detoxification of free heme [GO:0140725], GO:0140729, cellular detoxification [GO:1990748]